dolichyl-phosphate-mannose-protein mannosyltransferase complex [GO:0031502] (cellular component) Also known as: protein O-mannosyltransferase complex, PMT family mannosyltransferase complex Subtypes: dolichyl-phosphate-mannose-protein mannosyltransferase Pmt1p-Pmt2p dimer complex [GO:0097582], GO:0097583, dolichyl-phosphate-mannose-protein mannosyltransferase Pmt5p-Pmt2p dimer complex [GO:0097584], GO:0097585, dolichyl-phosphate-mannose-protein mannosyltransferase Pmt4p homodimer complex [GO:0097586] References: PMID:15948957 Sources: GOC:mah, GOC:pr Relationships: is a type of mannosyltransferase complex [GO:0031501]; is a type of GO:0098796; is a type of endoplasmic reticulum protein-containing complex [GO:0140534]; BFO_0000050 endoplasmic reticulum membrane [GO:0005789] Note: Note that GO:0004169 'dolichyl-phosphate-mannose-protein mannosyltransferase activity' (part of protein O-linked mannosylation) has never been observed in green plants. However, N- and C-mannosylation may occur in these species; see figure 1 in PMID:21558543. Definition: A complex that possesses dolichyl-phosphate-mannose-protein mannosyltransferase activity; usually includes members of the PMT1 and PMT2 protein subfamilies.